{
  "term_id": "GO:0045893",
  "term_label": "positive regulation of DNA-templated transcription",
  "gene_symbol": "LBH",
  "gene": "UniProtKB:Q53QV2",
  "gene_name": "Protein LBH"
}